{
  "gene_symbol": "KIF12",
  "term_label": "cytoplasm",
  "gene_name": "Kinesin-like protein KIF12",
  "term_id": "GO:0005737",
  "gene": "UniProtKB:Q96FN5"
}